{
  "gene": "UniProtKB:Q7Z695",
  "gene_symbol": "ADCK2",
  "term_label": "Unknown biological process",
  "gene_name": "Uncharacterized aarF domain-containing protein kinase 2",
  "term_id": "UNKNOWN:0002"
}